myosin XI tail binding [GO:0080115] (molecular function) Definition: Binding to the tail region of a myosin XI heavy chain. References: PMID:18703495 Relationships: is a type of myosin tail binding [GO:0032029]